{
  "term_label": "SUMO polymer binding",
  "gene": "UniProtKB:Q8NDZ2",
  "gene_symbol": "SIMC1",
  "term_id": "GO:0032184",
  "gene_name": "SUMO-interacting motif-containing protein 1"
}